{
  "gene": "UniProtKB:P59665",
  "term_label": "pore-forming activity",
  "gene_name": "Neutrophil defensin 1",
  "term_id": "GO:0140911",
  "gene_symbol": "DEFA1B"
}